serotonin secretion involved in inflammatory response [GO:0002442] (biological process) Subtypes: GO:0002552, serotonin secretion by platelet [GO:0002554], serotonin secretion by basophil [GO:0002556] Sources: GOC:add, ISBN:0781735149 Relationships: is a type of serotonin secretion [GO:0001820]; BFO_0000050 GO:0002351 Definition: The regulated release of serotonin by a cell as part of an inflammatory response. Also known as: serotonin secretion involved in acute inflammatory response, serotonin release involved in inflammatory response